{
  "gene_symbol": "KLHL6",
  "gene": "UniProtKB:Q8WZ60",
  "term_id": "GO:0031463",
  "gene_name": "Kelch-like protein 6",
  "term_label": "Cul3-RING ubiquitin ligase complex"
}